{
  "term_id": "GO:0005102",
  "gene_symbol": "FCN1",
  "gene_name": "Ficolin-1",
  "gene": "UniProtKB:O00602",
  "term_label": "signaling receptor binding"
}